{
  "term_id": "UNKNOWN:0003",
  "gene_name": "Coiled-coil domain-containing protein 142",
  "gene_symbol": "CCDC142",
  "term_label": "Unknown cellular component",
  "gene": "UniProtKB:Q17RM4"
}